{
  "term_label": "DNA-binding transcription factor activity, RNA polymerase II-specific",
  "gene": "UniProtKB:O60806",
  "term_id": "GO:0000981",
  "gene_symbol": "TBX19",
  "gene_name": "T-box transcription factor TBX19"
}